{
  "gene_name": "Zinc finger protein 18",
  "term_label": "Unknown cellular component",
  "term_id": "UNKNOWN:0003",
  "gene_symbol": "ZNF18",
  "gene": "UniProtKB:P17022"
}